tRNA pseudouridine(65) synthase activity [GO:0160149] (molecular function) Relationships: is a type of tRNA pseudouridine synthase activity [GO:0106029] Definition: Catalysis of the reaction: uridine(65) in tRNA = pseudouridine(65) in tRNA. Sources: EC:5.4.99.26